{
  "term_label": "actin monomer binding",
  "gene_name": "Myosin light chain 4",
  "term_id": "GO:0003785",
  "gene": "UniProtKB:P12829",
  "gene_symbol": "MYL4"
}